{
  "term_label": "Unknown biological process",
  "gene_symbol": "GAGE4",
  "gene_name": "G antigen 4",
  "term_id": "UNKNOWN:0002",
  "gene": "UniProtKB:P0DSO3"
}